{
  "gene_name": "Transcription initiation factor TFIID subunit 11",
  "gene": "UniProtKB:Q15544",
  "term_label": "transcription factor TFIID complex",
  "gene_symbol": "TAF11",
  "term_id": "GO:0005669"
}